{
  "term_label": "Unknown cellular component",
  "term_id": "UNKNOWN:0003",
  "gene": "UniProtKB:A0A0G2JND7",
  "gene_name": "Uncharacterized protein",
  "gene_symbol": "A0A0G2JND7"
}